{
  "gene_name": "Polycystin-1-like protein 1",
  "term_label": "calcium channel activity",
  "gene": "UniProtKB:Q8TDX9",
  "gene_symbol": "PKD1L1",
  "term_id": "GO:0005262"
}